{
  "gene": "UniProtKB:Q9NZI2",
  "gene_name": "Kv channel-interacting protein 1",
  "gene_symbol": "KCNIP1",
  "term_label": "potassium channel regulator activity",
  "term_id": "GO:0015459"
}